{
  "gene_name": "tRNA wybutosine-synthesizing protein 4",
  "gene": "UniProtKB:O60294",
  "term_id": "GO:0008175",
  "term_label": "tRNA methyltransferase activity",
  "gene_symbol": "LCMT2"
}